{
  "term_id": "UNKNOWN:0001",
  "gene_name": "NudC domain-containing protein 1",
  "term_label": "Unknown molecular function",
  "gene": "UniProtKB:Q96RS6",
  "gene_symbol": "NUDCD1"
}